{
  "term_label": "Unknown cellular component",
  "term_id": "UNKNOWN:0003",
  "gene_symbol": "SERTM1",
  "gene_name": "Serine-rich and transmembrane domain-containing protein 1",
  "gene": "UniProtKB:A2A2V5"
}